{
  "gene_name": "Ubiquitin-associated domain-containing protein 1",
  "term_id": "UNKNOWN:0002",
  "gene_symbol": "UBAC1",
  "gene": "UniProtKB:Q9BSL1",
  "term_label": "Unknown biological process"
}